{
  "gene": "UniProtKB:P48547",
  "gene_name": "Potassium voltage-gated channel subfamily C member 1",
  "term_label": "axon terminus",
  "gene_symbol": "KCNC1",
  "term_id": "GO:0043679"
}